{
  "term_label": "Unknown molecular function",
  "gene_symbol": "OR9A4",
  "term_id": "UNKNOWN:0001",
  "gene_name": "Olfactory receptor 9A4",
  "gene": "UniProtKB:Q8NGU2"
}